{
  "gene_name": "Probable non-functional T cell receptor beta variable 5-7",
  "gene": "UniProtKB:A0A0A0MS05",
  "term_id": "UNKNOWN:0001",
  "gene_symbol": "TRBV5-7",
  "term_label": "Unknown molecular function"
}